{
  "gene_name": "Heat shock 70 kDa protein 1-like",
  "term_label": "heat shock protein binding",
  "term_id": "GO:0031072",
  "gene_symbol": "HSPA1L",
  "gene": "UniProtKB:P34931"
}